{
  "gene_name": "Sphingosine kinase 2",
  "term_label": "sphingosine kinase activity",
  "gene": "UniProtKB:Q9NRA0",
  "term_id": "GO:0008481",
  "gene_symbol": "SPHK2"
}